{
  "term_label": "signal transduction",
  "gene_symbol": "ANGPT4",
  "gene": "UniProtKB:Q9Y264",
  "term_id": "GO:0007165",
  "gene_name": "Angiopoietin-4"
}